{
  "term_id": "UNKNOWN:0002",
  "gene_symbol": "A0A2R9YJI8",
  "term_label": "Unknown biological process",
  "gene": "UniProtKB:A0A2R9YJI8",
  "gene_name": "Uncharacterized protein"
}